atrial cardiac muscle cell action potential [GO:0086014] (biological process) Definition: An action potential that occurs in an atrial cardiac muscle cell. Sources: GOC:BHF, GOC:mtg_cardiac_conduct_nov11 Relationships: is a type of cardiac muscle cell action potential involved in contraction [GO:0086002]; BFO_0000050 GO:0086026 Regulation: regulated by regulation of atrial cardiac muscle cell action potential [GO:0098910]; negatively regulated by negative regulation of atrial cardiac muscle cell action potential [GO:1903948]; positively regulated by positive regulation of atrial cardiac muscle cell action potential [GO:1903949]